{
  "gene_symbol": "COA7",
  "term_id": "GO:0005758",
  "term_label": "mitochondrial intermembrane space",
  "gene_name": "Cytochrome c oxidase assembly factor 7",
  "gene": "UniProtKB:Q96BR5"
}